branch fusion, open tracheal system [GO:0035147] (biological process) Relationships: is a type of tube fusion [GO:0035146]; is part of branching involved in open tracheal system development [GO:0060446] Definition: Fusing of specific tracheal branches in an open tracheal system to branches from neighboring hemisegments to form a continuous tracheal network. Branch fusion is mediated by individual cells at the tip of each branch, which contact a similar cell and undergo a coordinated series of morphogenetic events that create a bicellular fusion joint. References: PMID:14570584 Sources: GOC:mtg_sensu Also known as: tracheal branch fusion